{
  "term_id": "GO:0005096",
  "gene": "UniProtKB:Q8WUA7",
  "gene_name": "TBC1 domain family member 22A",
  "term_label": "GTPase activator activity",
  "gene_symbol": "TBC1D22A"
}